precorrin-3B synthase activity [GO:0043818] (molecular function) Definition: Catalysis of the reaction: H+ + NADH + O2 + precorrin-3A = H2O + NAD+ + precorrin-3B. Relationships: is a type of oxidoreductase activity, acting on paired donors, with incorporation or reduction of molecular oxygen, NAD(P)H as one donor, and incorporation of one atom of oxygen [GO:0016709] Also known as: precorrin-3A,NADH:oxygen oxidoreductase (20-hydroxylating), CobG, precorrin-3X synthase activity Sources: EC:1.14.13.83, RHEA:17293